{
  "term_id": "GO:0061630",
  "gene_name": "F-box only protein 27",
  "term_label": "ubiquitin protein ligase activity",
  "gene_symbol": "FBXO27",
  "gene": "UniProtKB:Q8NI29"
}